{
  "gene_symbol": "MYO7B",
  "gene_name": "Unconventional myosin-VIIb",
  "gene": "UniProtKB:Q6PIF6",
  "term_label": "membrane",
  "term_id": "GO:0016020"
}